{
  "gene_name": "Protein-glutamine gamma-glutamyltransferase 5",
  "term_label": "Unknown cellular component",
  "term_id": "UNKNOWN:0003",
  "gene": "UniProtKB:O43548",
  "gene_symbol": "TGM5"
}